{
  "gene_symbol": "SEMA4B",
  "gene_name": "Semaphorin-4B",
  "term_id": "GO:0045499",
  "term_label": "chemorepellent activity",
  "gene": "UniProtKB:Q9NPR2"
}